AP-2 adaptor complex binding [GO:0035612] (MF) Definition: Binding to an AP-2 adaptor complex. The AP-2 adaptor complex is a heterotetrameric AP-type membrane coat adaptor complex that consists of alpha, beta2, mu2 and sigma2 subunits and links clathrin to the membrane surface of a vesicle. In at least humans, the AP-2 complex can be heterogeneric due to the existence of multiple subunit isoforms encoded by different alpha genes (alphaA and alphaC). Relationships: is_a protein-containing complex binding [GO:0044877] Also known as: AP-2 clathrin adaptor complex binding References: PMID:12221107, PMID:15728179, PMID:21097499 Sources: GOC:BHF